{
  "gene_symbol": "DLX2",
  "gene_name": "Homeobox protein DLX-2",
  "gene": "UniProtKB:Q07687",
  "term_label": "nucleus",
  "term_id": "GO:0005634"
}